{
  "term_label": "fatty acid biosynthetic process",
  "term_id": "GO:0006633",
  "gene": "UniProtKB:Q6NUN0",
  "gene_symbol": "ACSM5",
  "gene_name": "Acyl-coenzyme A synthetase ACSM5, mitochondrial"
}